negative regulation of peptide secretion [GO:0002792] (biological process) Subtypes: negative regulation of antimicrobial peptide secretion [GO:0002795], negative regulation of peptide hormone secretion [GO:0090278] Sources: GOC:add Also known as: down regulation of peptide secretion, down-regulation of peptide secretion, downregulation of peptide secretion, inhibition of peptide secretion Definition: Any process that stops, prevents, or reduces the frequency, rate, or extent of peptide secretion. Relationships: is a type of regulation of peptide secretion [GO:0002791]; is a type of negative regulation of secretion [GO:0051048]; negatively regulates peptide secretion [GO:0002790]